{
  "gene": "UniProtKB:O00159",
  "term_id": "GO:0051015",
  "gene_symbol": "MYO1C",
  "gene_name": "Unconventional myosin-Ic",
  "term_label": "actin filament binding"
}